{
  "gene_name": "ENTH domain-containing protein 1",
  "gene": "UniProtKB:Q8IYW4",
  "term_label": "clathrin binding",
  "term_id": "GO:0030276",
  "gene_symbol": "ENTHD1"
}